{
  "gene_name": "Tudor domain-containing protein 3",
  "gene": "UniProtKB:Q9H7E2",
  "term_label": "siRNA-mediated heterochromatin formation",
  "term_id": "GO:0141194",
  "gene_symbol": "TDRD3"
}